{
  "gene": "UniProtKB:Q9NP84",
  "term_label": "Unknown molecular function",
  "term_id": "UNKNOWN:0001",
  "gene_name": "Tumor necrosis factor receptor superfamily member 12A",
  "gene_symbol": "TNFRSF12A"
}